{
  "gene": "UniProtKB:P05451",
  "gene_name": "Lithostathine-1-alpha",
  "term_label": "antimicrobial humoral immune response mediated by antimicrobial peptide",
  "gene_symbol": "REG1A",
  "term_id": "GO:0061844"
}